type 2 somatostatin receptor binding [GO:0031879] (molecular function) Also known as: type 2 somatostatin receptor ligand Definition: Binding to a type 2 somatostatin receptor. Relationships: is a type of GO:0031877 Sources: GOC:mah, GOC:nln